{
  "gene": "UniProtKB:Q8WWN8",
  "term_id": "GO:0005547",
  "gene_symbol": "ARAP3",
  "term_label": "phosphatidylinositol-3,4,5-trisphosphate binding",
  "gene_name": "Arf-GAP with Rho-GAP domain, ANK repeat and PH domain-containing protein 3"
}